{
  "gene_symbol": "PCBP3",
  "term_id": "GO:0003729",
  "gene_name": "Poly(rC)-binding protein 3",
  "term_label": "mRNA binding",
  "gene": "UniProtKB:P57721"
}